{
  "gene_symbol": "CFAP184",
  "term_label": "ciliary basal body",
  "gene": "UniProtKB:Q2M329",
  "gene_name": "Coiled-coil domain-containing protein 96",
  "term_id": "GO:0036064"
}